positive regulation of granulocyte chemotaxis [GO:0071624] (biological process) Definition: Any process that increases the rate, frequency or extent of granulocyte chemotaxis. Granulocyte chemotaxis is the movement of a granulocyte in response to an external stimulus. Subtypes: positive regulation of neutrophil chemotaxis [GO:0090023], GO:2000424 Sources: GOC:mah Relationships: is a type of positive regulation of leukocyte chemotaxis [GO:0002690]; is a type of GO:0071622; positively regulates granulocyte chemotaxis [GO:0071621]